presynaptic endocytic zone cytoplasmic component [GO:0098834] (cellular component) Relationships: is_a GO:0099738; is part of GO:0098833 Also known as: cortex of presynaptic endocytic zone Sources: GOC:dos Definition: The cytoplasmic component of the presynaptic endocytic zone.